{
  "gene_symbol": "PCDHA6",
  "gene_name": "Protocadherin alpha-6",
  "term_label": "plasma membrane",
  "gene": "UniProtKB:Q9UN73",
  "term_id": "GO:0005886"
}